{
  "gene": "UniProtKB:O00468",
  "term_id": "GO:0007528",
  "term_label": "neuromuscular junction development",
  "gene_name": "Agrin",
  "gene_symbol": "AGRN"
}